regulation of peptidyl-tyrosine autophosphorylation [GO:1900084] (biological process) Subtypes: GO:1900085, positive regulation of peptidyl-tyrosine autophosphorylation [GO:1900086] Relationships: is a type of GO:0031952; is a type of regulation of peptidyl-tyrosine phosphorylation [GO:0050730]; regulates peptidyl-tyrosine autophosphorylation [GO:0038083] Sources: GOC:TermGenie, GOC:bf Also known as: regulation of tyrosine autophosphorylation, regulation of receptor tyrosine kinase autophosphorylation Definition: Any process that modulates the frequency, rate or extent of peptidyl-tyrosine autophosphorylation.